{
  "term_label": "Unknown biological process",
  "gene_symbol": "BMT2",
  "gene": "UniProtKB:Q1RMZ1",
  "gene_name": "S-adenosylmethionine sensor upstream of mTORC1",
  "term_id": "UNKNOWN:0002"
}